negative regulation of ovarian follicle development [GO:2000355] (biological process) Definition: Any process that stops, prevents or reduces the frequency, rate or extent of ovarian follicle development. Sources: GOC:obol Relationships: is_a GO:0051093; is a type of regulation of ovarian follicle development [GO:2000354]; negatively regulates ovarian follicle development [GO:0001541] Also known as: negative regulation of follicular phase